{
  "gene_symbol": "HLA-DQB1",
  "term_id": "GO:0042605",
  "term_label": "peptide antigen binding",
  "gene_name": "HLA class II histocompatibility antigen, DQ beta 1 chain",
  "gene": "UniProtKB:P01920"
}